{
  "gene_name": "Tyrosine-protein kinase Srms",
  "term_id": "GO:0005102",
  "gene": "UniProtKB:Q9H3Y6",
  "gene_symbol": "SRMS",
  "term_label": "signaling receptor binding"
}